{
  "term_id": "UNKNOWN:0001",
  "gene_name": "Golgin subfamily B member 1",
  "term_label": "Unknown molecular function",
  "gene": "UniProtKB:Q14789",
  "gene_symbol": "GOLGB1"
}